basal ring of apical complex [GO:0020032] (cellular component) Relationships: is a type of GO:0110165; is part of apical complex [GO:0020007] Definition: An electron dense ring at the most posterior position of the apical complex, from which the subpellicular microtubules originate; formed during an invasive life cycle stage of an apicomplexan parasite. Also known as: lower polar ring of apical complex, posterior polar ring of apical complex, preconoidal ring of apical complex References: PMID:16518471 Sources: GOC:mah